{
  "gene_name": "Fatty acid-binding protein, adipocyte",
  "term_id": "GO:0015908",
  "term_label": "fatty acid transport",
  "gene": "UniProtKB:P15090",
  "gene_symbol": "FABP4"
}